{
  "gene_name": "Ras and Rab interactor 2",
  "term_id": "GO:0005085",
  "gene_symbol": "RIN2",
  "term_label": "guanyl-nucleotide exchange factor activity",
  "gene": "UniProtKB:Q8WYP3"
}